{
  "term_label": "centrosome",
  "gene": "UniProtKB:Q9ULJ1",
  "gene_name": "Protein BCAP",
  "gene_symbol": "ODF2L",
  "term_id": "GO:0005813"
}